{
  "gene": "UniProtKB:A6NKF7",
  "term_label": "Unknown molecular function",
  "gene_name": "Transmembrane protein 88B",
  "term_id": "UNKNOWN:0001",
  "gene_symbol": "TMEM278"
}